{
  "gene": "UniProtKB:O15544",
  "gene_symbol": "LINC01565",
  "gene_name": "Protein GR6",
  "term_label": "Unknown molecular function",
  "term_id": "UNKNOWN:0001"
}